{
  "gene": "UniProtKB:Q16515",
  "gene_symbol": "ASIC2",
  "term_id": "GO:0005886",
  "gene_name": "Acid-sensing ion channel 2",
  "term_label": "plasma membrane"
}